{
  "gene_name": "Transcription factor Ovo-like 2",
  "term_id": "GO:0000981",
  "gene": "UniProtKB:Q9BRP0",
  "gene_symbol": "OVOL2",
  "term_label": "DNA-binding transcription factor activity, RNA polymerase II-specific"
}